{
  "gene_symbol": "PTPRS",
  "term_label": "synaptic membrane adhesion",
  "term_id": "GO:0099560",
  "gene_name": "Receptor-type tyrosine-protein phosphatase S",
  "gene": "UniProtKB:Q13332"
}